{
  "term_id": "GO:0006646",
  "gene_symbol": "CHKA",
  "term_label": "phosphatidylethanolamine biosynthetic process",
  "gene": "UniProtKB:P35790",
  "gene_name": "Choline kinase alpha"
}